bacterial-type flagellum [GO:0009288] (cellular component) Subtypes: GO:0055040 Also known as: flagellin-based flagellum Relationships: is a type of cell projection [GO:0042995]; is a type of membraneless organelle [GO:0043228] Definition: A motor complex composed of an extracellular helical protein filament coupled to a rotary motor embedded in the cell envelope. References: PMID:7787060 Sources: GOC:cilia, GOC:jh2, GOC:krc, GOC:mtg_sensu, Wikipedia:Flagellum#Bacterial